dystrobrevin complex [GO:0016014] (cellular component) Definition: A protein complex comprising alpha- and beta-dystrobrevin; forms part of the dystrophin glycoprotein complex. References: PMID:15117830, PMID:16710609 Relationships: is a type of GO:0098797; is part of dystrophin-associated glycoprotein complex [GO:0016010]